{
  "term_id": "GO:0035303",
  "gene_name": "Immunoglobulin-binding protein 1",
  "term_label": "regulation of dephosphorylation",
  "gene": "UniProtKB:P78318",
  "gene_symbol": "IGBP1"
}